homoserine O-succinyltransferase activity [GO:0008899] (molecular function) Also known as: homoserine O-transsuccinylase activity, homoserine succinyltransferase activity, succinyl-CoA:L-homoserine O-succinyltransferase activity Sources: EC:2.3.1.46, RHEA:22008 Relationships: is a type of GO:0016750 Definition: Catalysis of the reaction: L-homoserine + succinyl-CoA = O-succinyl-L-homoserine + CoA.